{
  "gene": "UniProtKB:Q9Y5G5",
  "term_id": "GO:0050839",
  "gene_name": "Protocadherin gamma-A8",
  "gene_symbol": "PCDHGA8",
  "term_label": "cell adhesion molecule binding"
}